{
  "term_label": "glucose-6-phosphate transport",
  "gene_symbol": "SLC37A1",
  "gene_name": "Glucose-6-phosphate exchanger SLC37A1",
  "term_id": "GO:0015760",
  "gene": "UniProtKB:P57057"
}